{
  "term_label": "nucleosomal DNA binding",
  "gene": "UniProtKB:P49450",
  "term_id": "GO:0031492",
  "gene_symbol": "CENPA",
  "gene_name": "Histone H3-like centromeric protein A"
}